{
  "term_label": "apical plasma membrane",
  "gene_name": "Podocalyxin",
  "gene_symbol": "PODXL",
  "term_id": "GO:0016324",
  "gene": "UniProtKB:O00592"
}